regulation of granulocyte differentiation [GO:0030852] (biological process) Relationships: is a type of regulation of myeloid leukocyte differentiation [GO:0002761]; regulates GO:0030851 Subtypes: negative regulation of granulocyte differentiation [GO:0030853], positive regulation of granulocyte differentiation [GO:0030854], regulation of basophil differentiation [GO:0045640], regulation of eosinophil differentiation [GO:0045643], regulation of neutrophil differentiation [GO:0045658] Definition: Any process that modulates the frequency, rate or extent of granulocyte differentiation. Sources: GOC:mah